establishment of blood-retinal barrier [GO:1990963] (biological process) Relationships: is_a cell development [GO:0048468] Definition: Establishment of the barrier between the blood and the retina. The blood-retinal barrier is located at two levels, forming an outer barrier in the retinal pigment epithelium and an inner barrier in the endothelial membrane of the retinal vessels. Both these membranes have tight junctions of the 'nonleaky' type. Also known as: establishment of blood-retina barrier, establishment of BRB References: PMID:25053619